{
  "term_id": "GO:0031430",
  "gene_symbol": "SMPX",
  "term_label": "M band",
  "gene": "UniProtKB:Q9UHP9",
  "gene_name": "Small muscular protein"
}